{
  "term_label": "cytosol",
  "term_id": "GO:0005829",
  "gene_symbol": "GOT1",
  "gene_name": "Aspartate aminotransferase, cytoplasmic",
  "gene": "UniProtKB:P17174"
}